miRNA transcription [GO:0061614] (biological process) Also known as: miRNA gene transcription, microRNA gene transcription, pri-miRNA transcription by RNA polymerase II, pri-miRNA transcription from RNA polymerase II promoter, primary miRNA gene transcription Definition: The cellular synthesis of microRNA (miRNA) transcripts. MicroRNA genes are synthesized as primary (pri) miRNA transcripts and subsequently processed to produce the ~22nt miRNAs that function in gene regulation. References: PMID:18778799 Sources: GOC:dph, GOC:kmv Regulation: regulated by GO:1902893; negatively regulated by negative regulation of miRNA transcription [GO:1902894]; positively regulated by positive regulation of miRNA transcription [GO:1902895] Relationships: is a type of DNA-templated transcription [GO:0006351]; is a type of GO:0010586